{
  "gene_symbol": "CLDN3",
  "gene_name": "Claudin-3",
  "gene": "UniProtKB:O15551",
  "term_label": "plasma membrane",
  "term_id": "GO:0005886"
}